{
  "gene_symbol": "POTEH",
  "gene_name": "POTE ankyrin domain family member H",
  "term_id": "UNKNOWN:0002",
  "gene": "UniProtKB:Q6S545",
  "term_label": "Unknown biological process"
}